{
  "term_id": "UNKNOWN:0003",
  "term_label": "Unknown cellular component",
  "gene": "UniProtKB:A0A8I5KTY6",
  "gene_symbol": "ZKSCAN8P1",
  "gene_name": "HCG1646484"
}